{
  "gene_name": "Zinc finger protein 837",
  "gene": "UniProtKB:Q96EG3",
  "term_id": "GO:0005634",
  "gene_symbol": "ZNF837",
  "term_label": "nucleus"
}